{
  "gene_name": "Pseudouridylate synthase PUS7L",
  "term_label": "pseudouridine synthase activity",
  "gene_symbol": "PUS7L",
  "gene": "UniProtKB:Q9H0K6",
  "term_id": "GO:0009982"
}